ferulate metabolic process [GO:0033494] (biological process) Sources: GOC:mah Definition: The chemical reactions and pathways involving ferulate, (2E)-3-(4-hydroxy-3-methoxyphenyl)prop-2-enoate. Relationships: is a type of phenol-containing compound metabolic process [GO:0018958]; is a type of monocarboxylic acid metabolic process [GO:0032787]; is a type of olefinic compound metabolic process [GO:0120254] Also known as: ferulate metabolism Subtypes: ferulate biosynthetic process [GO:0033495], ferulate catabolic process [GO:1901067]